{
  "gene": "UniProtKB:O00591",
  "term_label": "GABA-A receptor activity",
  "term_id": "GO:0004890",
  "gene_symbol": "GABRP",
  "gene_name": "Gamma-aminobutyric acid receptor subunit pi"
}